glutamyl-tRNA reductase activity [GO:0008883] (molecular function) Sources: EC:1.2.1.70, RHEA:12344 Also known as: L-glutamate-semialdehyde: NADP+ oxidoreductase (L-glutamyl-tRNAGlu-forming) Definition: Catalysis of the reaction: (S)-4-amino-5-oxopentanoate + NADP+ + tRNA(Glu) = L-glutamyl-tRNA(Glu) + H+ + NADPH. Relationships: is a type of GO:0016620; is_a GO:0140101